{
  "gene": "UniProtKB:P09493",
  "gene_name": "Tropomyosin alpha-1 chain",
  "term_id": "GO:0005884",
  "gene_symbol": "TPM1",
  "term_label": "actin filament"
}